{
  "term_id": "GO:0043235",
  "term_label": "receptor complex",
  "gene": "UniProtKB:P17948",
  "gene_name": "Vascular endothelial growth factor receptor 1",
  "gene_symbol": "FLT1"
}